{
  "term_label": "transmembrane transporter activity",
  "gene_name": "Anion exchange protein 3",
  "gene": "UniProtKB:P48751",
  "term_id": "GO:0022857",
  "gene_symbol": "SLC4A3"
}